D-tryptophan N-malonyltransferase activity [GO:0047836] (MF) Relationships: is_a GO:0050735 Definition: Catalysis of the reaction: D-tryptophan + malonyl-CoA = N(2)-malonyl-D-tryptophan + CoA + H+. Sources: EC:2.3.1.112, RHEA:23320 Also known as: malonyl-CoA:D-tryptophan N-malonyltransferase activity